{
  "gene_symbol": "MYLIP",
  "term_label": "Unknown cellular component",
  "term_id": "UNKNOWN:0003",
  "gene_name": "E3 ubiquitin-protein ligase MYLIP",
  "gene": "UniProtKB:Q8WY64"
}